{
  "gene_symbol": "DNAH10",
  "gene_name": "Dynein axonemal heavy chain 10",
  "term_id": "GO:0051959",
  "term_label": "dynein light intermediate chain binding",
  "gene": "UniProtKB:Q8IVF4"
}